neuron migration involved in retrograde extension [GO:0003393] (biological process) Sources: GOC:ascb_2009, GOC:dph, GOC:tb Definition: The directed, self-propelled movement of a neuron that contributes to the process of retrograde extension. Relationships: is a type of neuron migration [GO:0001764]; is part of retrograde extension [GO:0003389] Subtypes: neuron migration involved in dendrite retrograde extension [GO:0003395]